{
  "term_id": "GO:0017075",
  "gene_symbol": "STXBP3",
  "term_label": "syntaxin-1 binding",
  "gene": "UniProtKB:O00186",
  "gene_name": "Syntaxin-binding protein 3"
}